{
  "gene_symbol": "HIVEP2",
  "gene_name": "Transcription factor HIVEP2",
  "term_id": "GO:0000978",
  "term_label": "RNA polymerase II cis-regulatory region sequence-specific DNA binding",
  "gene": "UniProtKB:P31629"
}